regulation of mesenchymal cell proliferation involved in lung development [GO:2000790] (biological process) References: PMID:21513708 Subtypes: negative regulation of mesenchymal cell proliferation involved in lung development [GO:2000791], GO:2000792 Relationships: is a type of regulation of mesenchymal cell proliferation [GO:0010464]; regulates mesenchymal cell proliferation involved in lung development [GO:0060916] Definition: Any process that modulates the frequency, rate or extent of mesenchymal cell proliferation involved in lung development.